N-methylnicotinate transmembrane transporter activity [GO:0090417] (molecular function) Sources: GOC:tb Relationships: is a type of GO:0015651; is part of N-methylnicotinate transport [GO:2001143] Also known as: N-methylnicotinate transporter activity Definition: Enables the transfer of N-methylnicotinate from one side of a membrane to the other.